{
  "gene_symbol": "ADGRG2",
  "gene": "UniProtKB:Q8IZP9",
  "gene_name": "Adhesion G-protein coupled receptor G2",
  "term_id": "GO:0007186",
  "term_label": "G protein-coupled receptor signaling pathway"
}